{
  "gene_symbol": "RNF222",
  "gene": "UniProtKB:A6NCQ9",
  "term_label": "Unknown molecular function",
  "term_id": "UNKNOWN:0001",
  "gene_name": "RING finger protein 222"
}